cross bridge formation involved in regulation of the velocity of shortening in skeletal muscle contraction [GO:0014871] (biological process) Relationships: is a type of regulation of muscle filament sliding involved in regulation of the velocity of shortening in skeletal muscle contraction [GO:0014880] Sources: GOC:mtg_muscle Definition: The process in which actin and myosin interact, split ATP and generate force during skeletal muscle contraction. This process is one of the components of the regulation of the force of skeletal muscle contraction.